neural crest-derived cardiac glial cell fate commitment [GO:0060955] (biological process) Relationships: is a type of cardiac glial cell fate commitment [GO:0060953]; is part of GO:0060951 Definition: The commitment of neural crest cells to cardiac glial cell fates and their capacity to differentiate into cardiac glial cells. Sources: GOC:mtg_heart